{
  "gene": "UniProtKB:P50552",
  "term_label": "positive regulation of actin filament polymerization",
  "term_id": "GO:0030838",
  "gene_name": "Vasodilator-stimulated phosphoprotein",
  "gene_symbol": "VASP"
}